negative regulation of epithelial tube formation [GO:1905277] (biological process) References: PMID:25745997 Sources: GOC:TermGenie, GOC:bhm, GO_REF:0000058 Definition: Any process that stops, prevents or reduces the frequency, rate or extent of epithelial tube formation. Relationships: is a type of negative regulation of multicellular organismal process [GO:0051241]; is a type of regulation of epithelial tube formation [GO:1905276]; is a type of negative regulation of morphogenesis of an epithelium [GO:1905331]; negatively regulates epithelial tube formation [GO:0072175] Also known as: down regulation of epithelial tube formation, down-regulation of epithelial tube formation, downregulation of epithelial tube formation, inhibition of epithelial tube formation Note: An example of this is MMRN2 in human (Q9H8L6) in PMID:25745997 (inferred from direct assay).